coenzyme A binding [GO:0120225] (molecular function) Relationships: is a type of amide binding [GO:0033218]; is a type of anion binding [GO:0043168]; is a type of nucleoside phosphate binding [GO:1901265]; is a type of GO:1901363; is a type of sulfur compound binding [GO:1901681] Sources: GOC:krc, ISBN:0198547684 Also known as: CoA binding Definition: Binding to coenzyme A, 3'-phosphoadenosine-(5')diphospho(4')pantatheine, an acyl carrier in many acylation and acyl-transfer reactions in which the intermediate is a thiol ester.